{
  "gene_symbol": "ACVR2B",
  "gene": "UniProtKB:Q13705",
  "term_id": "GO:0005886",
  "term_label": "plasma membrane",
  "gene_name": "Activin receptor type-2B"
}